{
  "gene": "UniProtKB:Q3KNV8",
  "term_id": "GO:0006357",
  "term_label": "regulation of transcription by RNA polymerase II",
  "gene_name": "Polycomb group RING finger protein 3",
  "gene_symbol": "PCGF3"
}